{
  "gene_name": "Inactive ubiquitin carboxyl-terminal hydrolase 53",
  "gene": "UniProtKB:Q70EK8",
  "term_label": "Unknown molecular function",
  "gene_symbol": "USP53",
  "term_id": "UNKNOWN:0001"
}